{
  "gene_name": "Gamma-adducin",
  "term_id": "GO:0051016",
  "gene_symbol": "ADD3",
  "term_label": "barbed-end actin filament capping",
  "gene": "UniProtKB:Q9UEY8"
}